{
  "term_id": "GO:0005262",
  "term_label": "calcium channel activity",
  "gene_name": "Growth hormone-inducible transmembrane protein",
  "gene_symbol": "GHITM",
  "gene": "UniProtKB:Q9H3K2"
}